G2/MI transition of meiotic cell cycle [GO:0008315] (biological process) Relationships: is_a meiotic cell cycle phase transition [GO:0044771]; is a type of cell cycle G2/M phase transition [GO:0044839]; is a type of GO:0061982 References: PMID:15084480 Regulation: regulated by regulation of G2/MI transition of meiotic cell cycle [GO:0110030]; negatively regulated by negative regulation of G2/MI transition of meiotic cell cycle [GO:0110031]; positively regulated by positive regulation of G2/MI transition of meiotic cell cycle [GO:0110032] Definition: The cell cycle process in which a cell progresses from meiotic G2 phase to M phase of meiosis I. Also known as: meiotic G2/MI phase transition, meiotic G2/MI transition, meiotic cell cycle G2/MI phase transition